urea transmembrane transporter activity [GO:0015204] (molecular function) Also known as: urea transporter activity Sources: ISBN:0198506732 Definition: Enables the transfer of urea from one side of a membrane to the other. Urea is the water soluble compound H2N-CO-NH2. Relationships: is a type of amide transmembrane transporter activity [GO:0042887]; is part of urea transmembrane transport [GO:0071918] Subtypes: urea channel activity [GO:0015265], urea:sodium symporter activity [GO:0015401], ATPase-coupled urea transmembrane transporter activity [GO:0033221]